{
  "gene_name": "Uncharacterized protein C14orf93",
  "gene_symbol": "C14orf93",
  "term_label": "Unknown molecular function",
  "gene": "UniProtKB:Q9H972",
  "term_id": "UNKNOWN:0001"
}